heterochromatin [GO:0000792] (cellular component) Also known as: transcriptionally inactive chromatin, transcriptionally silent chromatin, nuclear heterochromatin Subtypes: GO:0001739, pericentric heterochromatin [GO:0005721], intercalary heterochromatin [GO:0005725], mating-type region heterochromatin [GO:0031934], GO:0033553, senescence-associated heterochromatin focus [GO:0035985], GO:0140720, heterochromatin island [GO:1990342], heterochromatin domain [GO:1990343] Relationships: is_a chromatin [GO:0000785] References: PMID:32017156 Definition: A compact and highly condensed form of chromatin that is refractory to transcription.